{
  "gene": "UniProtKB:P61254",
  "term_label": "RNA binding",
  "gene_name": "Large ribosomal subunit protein uL24",
  "gene_symbol": "RPL26",
  "term_id": "GO:0003723"
}